{
  "gene": "UniProtKB:Q12951",
  "gene_symbol": "FOXI1",
  "term_id": "GO:0030154",
  "term_label": "cell differentiation",
  "gene_name": "Forkhead box protein I1"
}